response to haloperidol [GO:1905119] (biological process) Definition: Any process that results in a change in state or activity of a cell or an organism (in terms of movement, secretion, enzyme production, gene expression, etc.) as a result of a haloperidol stimulus. References: PMID:24751813 Sources: GOC:TermGenie, GOC:dw, GO_REF:0000071 Note: Note that this term is in the subset of terms that should not be used for direct manual annotation of gene products. It was created to be used for cross-referencing by other ontologies. Direct annotations to this term may be amended during annotation QC. Relationships: is a type of response to alcohol [GO:0097305]; is a type of response to ketone [GO:1901654]; is a type of response to nitrogen compound [GO:1901698] Subtypes: cellular response to haloperidol [GO:1905120]